{
  "term_label": "9+2 motile cilium",
  "term_id": "GO:0097729",
  "gene": "UniProtKB:Q9P225",
  "gene_symbol": "DNAH2",
  "gene_name": "Dynein axonemal heavy chain 2"
}